{
  "term_label": "endomembrane system",
  "gene_name": "Protein O-glucosyltransferase 1",
  "term_id": "GO:0012505",
  "gene_symbol": "POGLUT1",
  "gene": "UniProtKB:Q8NBL1"
}